{
  "term_label": "ubiquitin protein ligase activity",
  "gene_symbol": "RNF181",
  "gene_name": "E3 ubiquitin-protein ligase RNF181",
  "gene": "UniProtKB:Q9P0P0",
  "term_id": "GO:0061630"
}